cone matrix sheath [GO:0090658] (CC) Definition: A biochemically and structurally distinct domain of the retinal interphotoreceptor matrix that is specifically associated with cone photoreceptor cell inner and outer segments. References: PMID:2055688 Sources: GOC:mr Relationships: is a type of cellular anatomical structure [GO:0110165]; BFO_0000050 GO:0033165